{
  "gene_symbol": "SHLD1",
  "gene_name": "Shieldin complex subunit 1",
  "term_id": "GO:2001034",
  "gene": "UniProtKB:Q8IYI0",
  "term_label": "positive regulation of double-strand break repair via nonhomologous end joining"
}